{
  "term_id": "GO:0031593",
  "term_label": "polyubiquitin modification-dependent protein binding",
  "gene": "UniProtKB:Q6UWZ7",
  "gene_symbol": "ABRAXAS1",
  "gene_name": "BRCA1-A complex subunit Abraxas 1"
}